{
  "term_label": "DNA-binding transcription factor activity, RNA polymerase II-specific",
  "gene": "UniProtKB:Q96NL3",
  "gene_name": "Zinc finger protein 599",
  "term_id": "GO:0000981",
  "gene_symbol": "ZNF599"
}